neuropeptide Y receptor activity [GO:0004983] (molecular function) Relationships: is a type of neuropeptide receptor activity [GO:0008188] Subtypes: peptide YY receptor activity [GO:0001601], pancreatic polypeptide receptor activity [GO:0001602] References: PMID:9315606 Definition: Combining with neuropeptide Y to initiate a change in cell activity.